{
  "gene_symbol": "RAB17",
  "term_label": "plasma membrane",
  "gene_name": "Ras-related protein Rab-17",
  "gene": "UniProtKB:Q9H0T7",
  "term_id": "GO:0005886"
}